{
  "gene": "UniProtKB:O00566",
  "gene_symbol": "MPHOSPH10",
  "gene_name": "U3 small nucleolar ribonucleoprotein protein MPP10",
  "term_label": "small-subunit processome",
  "term_id": "GO:0032040"
}